{
  "gene_name": "Organic anion transporter 3",
  "gene": "UniProtKB:Q8TCC7",
  "gene_symbol": "SLC22A8",
  "term_id": "UNKNOWN:0001",
  "term_label": "Unknown molecular function"
}